{
  "gene_name": "Oxysterols receptor LXR-alpha",
  "term_id": "GO:0005634",
  "gene_symbol": "NR1H3",
  "term_label": "nucleus",
  "gene": "UniProtKB:Q13133"
}